{
  "gene": "UniProtKB:Q96LJ8",
  "gene_name": "UBX domain-containing protein 10",
  "term_id": "GO:0036503",
  "term_label": "ERAD pathway",
  "gene_symbol": "UBXN10"
}